{
  "term_id": "GO:0016477",
  "term_label": "cell migration",
  "gene": "UniProtKB:O00507",
  "gene_name": "Probable ubiquitin carboxyl-terminal hydrolase FAF-Y",
  "gene_symbol": "USP9Y"
}